{
  "gene_name": "Histidine decarboxylase",
  "term_label": "L-histidine catabolic process",
  "gene": "UniProtKB:P19113",
  "gene_symbol": "HDC",
  "term_id": "GO:0006548"
}